{
  "gene_symbol": "BCL2L2",
  "gene_name": "Bcl-2-like protein 2",
  "term_label": "positive regulation of apoptotic process",
  "gene": "UniProtKB:Q92843",
  "term_id": "GO:0043065"
}